{
  "gene_name": "Phosphatidylinositol N-acetylglucosaminyltransferase subunit H",
  "term_id": "GO:0000506",
  "gene_symbol": "PIGH",
  "term_label": "glycosylphosphatidylinositol-N-acetylglucosaminyltransferase (GPI-GnT) complex",
  "gene": "UniProtKB:Q14442"
}